regulation of response to pullulan [GO:1900518] (biological process) Relationships: is a type of regulation of response to stimulus [GO:0048583]; regulates response to pullulan [GO:0044592] Subtypes: negative regulation of response to pullulan [GO:1900519], positive regulation of response to pullulan [GO:1900520] Sources: GOC:TermGenie, GOC:mengo_curators Definition: Any process that modulates the frequency, rate or extent of response to pullulan.